{
  "gene_symbol": "GOSR2",
  "gene_name": "Golgi SNAP receptor complex member 2",
  "term_id": "GO:0012507",
  "gene": "UniProtKB:O14653",
  "term_label": "ER to Golgi transport vesicle membrane"
}